{
  "gene_symbol": "AAGAB",
  "gene_name": "Alpha- and gamma-adaptin-binding protein p34",
  "gene": "UniProtKB:Q6PD74",
  "term_label": "Unknown cellular component",
  "term_id": "UNKNOWN:0003"
}